{
  "term_id": "UNKNOWN:0003",
  "gene": "UniProtKB:Q9BXY5",
  "term_label": "Unknown cellular component",
  "gene_name": "Calcyphosin-2",
  "gene_symbol": "CAPS2"
}